DNA polymerase III complex [GO:0009360] (cellular component) Relationships: is a type of GO:0042575 References: PMID:11525729, PMID:12940977 Sources: UniProt:P06710 Definition: The DNA polymerase III holoenzyme is a complex that contains 10 different types of subunits. These subunits are organized into 3 functionally essential sub-assemblies: the pol III core, the beta sliding clamp processivity factor and the clamp-loading complex. The pol III core carries out the polymerase and the 3'-5' exonuclease proofreading activities. The polymerase is tethered to the template via the sliding clamp processivity factor. The clamp-loading complex assembles the beta processivity factor onto the primer template and plays a central role in the organization and communication at the replication fork. Also known as: DNA polymerase III holoenzyme complex